actin filament depolymerization [GO:0030042] (biological process) Sources: GOC:mah Relationships: is a type of GO:0008154; is a type of protein depolymerization [GO:0051261] Subtypes: GO:0030043 Definition: Disassembly of actin filaments by the removal of actin monomers from a filament. Also known as: actin depolymerization, actin depolymerizing activity Regulation: regulated by regulation of actin filament depolymerization [GO:0030834]; negatively regulated by negative regulation of actin filament depolymerization [GO:0030835]; positively regulated by positive regulation of actin filament depolymerization [GO:0030836]